glycoside biosynthetic process [GO:0016138] (biological process) Definition: The chemical reactions and pathways resulting in the formation of glycosides, compounds in which a glycosyl group is substituted into a hydroxyl, thiol or selenol group in another compound. Sources: GOC:go_curators Also known as: O-glycoside anabolism, O-glycoside biosynthesis, O-glycoside biosynthetic process, O-glycoside formation, O-glycoside synthesis, glycoside anabolism, glycoside biosynthesis, glycoside formation, glycoside synthesis Relationships: is a type of GO:0016137; is a type of glycosyl compound biosynthetic process [GO:1901659] Subtypes: GO:0010125, saponin biosynthetic process [GO:0016135], cyanogenic glycoside biosynthetic process [GO:0019756], aminoglycoside antibiotic biosynthetic process [GO:0030648], quercetin O-glucoside biosynthetic process [GO:0033303], novobiocin biosynthetic process [GO:0043642], glucosylglycerol biosynthetic process [GO:0051473], mannosylglycerate biosynthetic process [GO:0051479], bacillithiol biosynthetic process [GO:0071793], tobramycin biosynthetic process [GO:1901121], butirosin biosynthetic process [GO:1901758], GO:1901806, ascaroside biosynthetic process [GO:1904070]